{
  "term_id": "GO:0000045",
  "gene": "UniProtKB:O95166",
  "gene_name": "Gamma-aminobutyric acid receptor-associated protein",
  "term_label": "autophagosome assembly",
  "gene_symbol": "GABARAP"
}